cardiac neural crest cell development involved in heart development [GO:0061308] (biological process) Relationships: is a type of neural crest cell development [GO:0014032]; is part of cardiac neural crest cell differentiation involved in heart development [GO:0061307] Sources: GOC:dph, GOC:mtg_heart Definition: The process aimed at the progression of a cardiac neural crest cell over time, from initial commitment of the cell to its specific fate, to the fully functional differentiated cell that contributes to the development of the heart. Subtypes: cardiac neural crest cell development involved in outflow tract morphogenesis [GO:0061309]